type I terminal bouton [GO:0061174] (cellular component) Sources: GOC:dph, GOC:mc Definition: Terminal inflated portion of the axon of a glutamatergic neuron, containing the specialized apparatus necessary to release neurotransmitters that will induce the contraction of muscle. The axon terminus is considered to be the whole region of thickening and the terminal bouton is a specialized region of it. Also known as: type I terminal button Subtypes: type Ib terminal bouton [GO:0061176], type Is terminal bouton [GO:0061177] Relationships: is a type of terminal bouton [GO:0043195]